{
  "gene_symbol": "GRID1",
  "term_label": "AMPA glutamate receptor activity",
  "gene": "UniProtKB:Q9ULK0",
  "gene_name": "Glutamate receptor ionotropic, delta-1",
  "term_id": "GO:0004971"
}